protein-carbohydrate complex disassembly [GO:0032985] (biological process) Sources: GOC:mah Relationships: is a type of protein-containing complex disassembly [GO:0032984]; is a type of GO:0071823 Definition: The disaggregation of a protein-carbohydrate complex into its constituent components.